{
  "gene_name": "T-cell surface antigen CD2",
  "term_id": "GO:0006955",
  "gene_symbol": "CD2",
  "gene": "UniProtKB:P06729",
  "term_label": "immune response"
}